{
  "gene_symbol": "RAF1",
  "gene": "UniProtKB:P04049",
  "gene_name": "RAF proto-oncogene serine_threonine-protein kinase",
  "term_id": "GO:0000165",
  "term_label": "MAPK cascade"
}